{
  "gene_name": "Olfactory receptor 14I1",
  "gene_symbol": "OR14I1",
  "term_label": "odorant binding",
  "gene": "UniProtKB:A6ND48",
  "term_id": "GO:0005549"
}